pantothenate transmembrane transport [GO:0015887] (biological process) Definition: The process in which pantothenate is transported across a membrane. Pantothenate is the anion of pantothenic acid, the amide of beta-alanine and pantoic acid; it is a B complex vitamin that is a constituent of coenzyme A and is distributed ubiquitously in foods. Also known as: pantothenate membrane transport, pantothenate transport, vitamin B5 transport Note: Note that this term is not intended for use in annotating lateral movement within membranes. Subtypes: pantothenate import across plasma membrane [GO:0098717] Sources: GOC:ai, ISBN:0721662544 Relationships: is a type of monocarboxylic acid transport [GO:0015718]; is a type of vitamin transmembrane transport [GO:0035461]; is a type of amide transport [GO:0042886]; is_a modified amino acid transport [GO:0072337]; is a type of carboxylic acid transmembrane transport [GO:1905039]